{
  "term_id": "GO:0000724",
  "term_label": "double-strand break repair via homologous recombination",
  "gene_symbol": "KAT5",
  "gene_name": "Histone acetyltransferase KAT5",
  "gene": "UniProtKB:Q92993"
}